denitrification pathway [GO:0019333] (biological process) Definition: The reduction of nitrate to dinitrogen by four reduction reactions: nitrate reduced to nitrite, then to nitric oxide, then to nitrous oxide, and finally to dinitrogen. Sources: MetaCyc:DENITRIFICATION-PWY Relationships: is a type of nitrogen cycle metabolic process [GO:0071941]; has part GO:0008940; has part GO:0050304